{
  "gene_name": "Protein lin-37 homolog",
  "term_label": "Unknown molecular function",
  "gene": "UniProtKB:Q96GY3",
  "term_id": "UNKNOWN:0001",
  "gene_symbol": "LIN37"
}